{
  "term_id": "GO:0016324",
  "gene_symbol": "SLCO2B1",
  "gene_name": "Solute carrier organic anion transporter family member 2B1",
  "gene": "UniProtKB:O94956",
  "term_label": "apical plasma membrane"
}